tRNA transport [GO:0051031] (biological process) Definition: The directed movement of tRNA, transfer ribonucleic acid, into, out of or within a cell, or between cells, by means of some agent such as a transporter or pore. Relationships: is a type of RNA transport [GO:0050658] Subtypes: tRNA export from nucleus [GO:0006409], tRNA import into mitochondrion [GO:0016031], tRNA import into nucleus [GO:0035719] Sources: GOC:ai